{
  "gene": "UniProtKB:P48730",
  "gene_name": "Casein kinase I isoform delta",
  "term_label": "endocytosis",
  "term_id": "GO:0006897",
  "gene_symbol": "CSNK1D"
}